Spemann organizer formation at the anterior end of the primitive streak [GO:0060064] (biological process) Definition: Formation of the specialized region at the anterior end of the primitive streak of the embryo that acts as the main signaling center establishing the body plan. References: PMID:9442883 Sources: GOC:dph Also known as: Spemann's organizer formation at the anterior end of the primitive streak, Spemann organizer formation in amniotes, Spemann-Mangold organizer formation at the anterior end of the primitive streak Note: Occurs in reptiles, birds and mammals. Relationships: is a type of Spemann organizer formation [GO:0060061]